{
  "gene": "UniProtKB:H0Y7S4",
  "gene_name": "Putative PRAME family member 26",
  "term_label": "Cul2-RING ubiquitin ligase complex",
  "gene_symbol": "PRAMEF26",
  "term_id": "GO:0031462"
}